{
  "gene_name": "Sodium channel protein type 9 subunit alpha",
  "term_id": "GO:0005248",
  "gene_symbol": "SCN9A",
  "term_label": "voltage-gated sodium channel activity",
  "gene": "UniProtKB:Q15858"
}